{
  "gene": "UniProtKB:Q701N2",
  "term_label": "Unknown molecular function",
  "term_id": "UNKNOWN:0001",
  "gene_symbol": "KRTAP5-5",
  "gene_name": "Keratin-associated protein 5-5"
}